{
  "gene": "UniProtKB:Q7Z7J5",
  "term_id": "GO:0005634",
  "term_label": "nucleus",
  "gene_symbol": "DPPA2",
  "gene_name": "Developmental pluripotency-associated protein 2"
}